{
  "term_id": "GO:0000786",
  "gene_symbol": "H2AC7",
  "gene_name": "Histone H2A type 1-D",
  "gene": "UniProtKB:P20671",
  "term_label": "nucleosome"
}